{
  "gene_name": "Periplakin",
  "term_id": "GO:0005198",
  "term_label": "structural molecule activity",
  "gene_symbol": "PPL",
  "gene": "UniProtKB:O60437"
}